{
  "gene_symbol": "KCNS1",
  "gene": "UniProtKB:Q96KK3",
  "term_id": "GO:0071805",
  "term_label": "potassium ion transmembrane transport",
  "gene_name": "Potassium voltage-gated channel subfamily S member 1"
}